regulation of hydrogen peroxide-mediated programmed cell death [GO:1901298] (biological process) Relationships: is_a regulation of programmed cell death [GO:0043067]; regulates hydrogen peroxide-mediated programmed cell death [GO:0010421] Subtypes: negative regulation of hydrogen peroxide-mediated programmed cell death [GO:1901299], GO:1901300, regulation of intrinsic apoptotic signaling pathway in response to hydrogen peroxide [GO:1903750] Definition: Any process that modulates the frequency, rate or extent of hydrogen peroxide-mediated programmed cell death. Sources: GOC:BHF, GOC:TermGenie